{
  "gene_symbol": "PPARA",
  "term_id": "GO:0009755",
  "gene": "UniProtKB:Q07869",
  "gene_name": "Peroxisome proliferator-activated receptor alpha",
  "term_label": "hormone-mediated signaling pathway"
}